{
  "term_id": "GO:0005737",
  "gene": "UniProtKB:Q8WVZ7",
  "term_label": "cytoplasm",
  "gene_symbol": "RNF133",
  "gene_name": "E3 ubiquitin-protein ligase RNF133"
}